{
  "term_label": "extracellular space",
  "gene_name": "Cathepsin B",
  "term_id": "GO:0005615",
  "gene": "UniProtKB:P07858",
  "gene_symbol": "CTSB"
}